GABAergic neuron differentiation [GO:0097154] (biological process) Definition: The process in which a neuroblast acquires the specialized structural and functional features of a GABAergic neuron. Subtypes: cerebellar Golgi cell differentiation [GO:0021701], GO:0021708, GO:0021773, GABAergic neuron differentiation in basal ganglia [GO:0021858], cerebral cortex GABAergic interneuron differentiation [GO:0021892] References: PMID:11517269 Sources: GOC:kmv Relationships: is a type of neuron differentiation [GO:0030182]